{
  "gene": "UniProtKB:P32189",
  "gene_symbol": "GK",
  "term_label": "mitochondrion",
  "term_id": "GO:0005739",
  "gene_name": "Glycerol kinase"
}